positive regulation of single-species biofilm formation on inanimate substrate [GO:1900233] (biological process) Definition: Any process that activates or increases the frequency, rate or extent of single-species biofilm formation on inanimate substrate. Sources: GOC:TermGenie, GOC:di Also known as: up regulation of single-species biofilm formation on inanimate substrate, up-regulation of single-species biofilm formation on inanimate substrate, upregulation of single-species biofilm formation on inanimate substrate, activation of single-species biofilm formation on inanimate substrate Relationships: is a type of positive regulation of single-species biofilm formation [GO:1900192]; is a type of GO:1900231; RO_0002213 single-species biofilm formation on inanimate substrate [GO:0044011]